{
  "term_id": "UNKNOWN:0003",
  "gene_name": "C-X-C motif chemokine 2",
  "gene_symbol": "CXCL2",
  "term_label": "Unknown cellular component",
  "gene": "UniProtKB:P19875"
}